{
  "gene_symbol": "C9orf78",
  "term_id": "GO:0005681",
  "term_label": "spliceosomal complex",
  "gene_name": "Splicing factor C9orf78",
  "gene": "UniProtKB:Q9NZ63"
}